{
  "gene": "UniProtKB:P49747",
  "term_id": "UNKNOWN:0002",
  "term_label": "Unknown biological process",
  "gene_name": "Cartilage oligomeric matrix protein",
  "gene_symbol": "COMP"
}